positive regulation of acrosome reaction [GO:2000344] (biological process) Relationships: is a type of regulation of acrosome reaction [GO:0060046]; is a type of positive regulation of reproductive process [GO:2000243]; RO_0002213 acrosome reaction [GO:0007340] Definition: Any process that activates or increases the frequency, rate or extent of the acrosome reaction. Sources: GOC:obol